fatty alcohol biosynthetic process [GO:1903175] (biological process) Definition: The chemical reactions and pathways resulting in the formation of fatty alcohol. References: PMID:24036493 Sources: GOC:TermGenie, GOC:mengo_curators, GO_REF:0000068 Also known as: fatty alcohol anabolism, fatty alcohol biosynthesis, fatty alcohol formation, fatty alcohol synthesis Relationships: is_a alcohol biosynthetic process [GO:0046165]; is a type of fatty acid derivative biosynthetic process [GO:1901570]; is a type of GO:1903173 Subtypes: phytol biosynthetic process [GO:0033520], octanol biosynthetic process [GO:0046171], 1-butanol biosynthetic process [GO:0071271], propan-2-ol biosynthetic process [GO:1902640]